{
  "gene_symbol": "ZNF532",
  "term_id": "UNKNOWN:0002",
  "gene_name": "Zinc finger protein 532",
  "gene": "UniProtKB:Q9HCE3",
  "term_label": "Unknown biological process"
}